superior reticular formation development [GO:0021729] (biological process) Sources: GOC:cls, GOC:curators, GOC:dgh, GOC:dph, GOC:jid Definition: The process whose specific outcome is the progression of the superior reticular formation over time, from its formation to the mature structure. Relationships: is a type of anatomical structure development [GO:0048856]; is part of medullary reticular formation development [GO:0021723]